{
  "gene": "UniProtKB:Q9H3V2",
  "gene_symbol": "MS4A5",
  "gene_name": "Membrane-spanning 4-domains subfamily A member 5",
  "term_id": "UNKNOWN:0001",
  "term_label": "Unknown molecular function"
}